positive regulation of low-density lipoprotein particle clearance [GO:1905581] (biological process) Definition: Any process that activates or increases the frequency, rate or extent of low-density lipoprotein particle clearance. References: PMID:22848640 Sources: GOC:BHF, GOC:TermGenie, GOC:nc, GO_REF:0000058 Also known as: positive regulation of LDL clearance, up regulation of LDL clearance, up regulation of low-density lipoprotein particle clearance, up-regulation of LDL clearance, up-regulation of low-density lipoprotein particle clearance, upregulation of LDL clearance, upregulation of low-density lipoprotein particle clearance, activation of LDL clearance, activation of low-density lipoprotein particle clearance Relationships: is a type of positive regulation of lipoprotein particle clearance [GO:0010986]; is a type of regulation of low-density lipoprotein particle clearance [GO:0010988]; positively regulates low-density lipoprotein particle clearance [GO:0034383]